{
  "term_id": "UNKNOWN:0001",
  "gene": "UniProtKB:Q9UF11",
  "term_label": "Unknown molecular function",
  "gene_name": "Pleckstrin homology domain-containing family B member 1",
  "gene_symbol": "PLEKHB1"
}